{
  "gene_name": "Mitogen-activated protein kinase 15",
  "term_id": "GO:0005634",
  "gene": "UniProtKB:Q8TD08",
  "term_label": "nucleus",
  "gene_symbol": "MAPK15"
}